{
  "gene": "UniProtKB:Q7Z6K1",
  "term_id": "UNKNOWN:0001",
  "term_label": "Unknown molecular function",
  "gene_symbol": "THAP5",
  "gene_name": "THAP domain-containing protein 5"
}